{
  "term_label": "Unknown molecular function",
  "gene_symbol": "C17orf75",
  "term_id": "UNKNOWN:0001",
  "gene": "UniProtKB:Q9HAS0",
  "gene_name": "Protein Njmu-R1"
}